{
  "term_id": "GO:0005886",
  "gene_name": "Olfactory receptor 51E1",
  "gene": "UniProtKB:Q8TCB6",
  "gene_symbol": "OR51E1",
  "term_label": "plasma membrane"
}